{
  "gene": "UniProtKB:P48065",
  "gene_name": "Sodium- and chloride-dependent betaine transporter",
  "gene_symbol": "SLC6A12",
  "term_label": "plasma membrane",
  "term_id": "GO:0005886"
}